{
  "term_label": "sphingosine biosynthetic process",
  "gene_name": "Serine palmitoyltransferase 1",
  "gene": "UniProtKB:O15269",
  "term_id": "GO:0046512",
  "gene_symbol": "SPTLC1"
}